{
  "gene": "UniProtKB:Q6S8J3",
  "term_id": "GO:0015629",
  "gene_name": "POTE ankyrin domain family member E",
  "term_label": "actin cytoskeleton",
  "gene_symbol": "POTEE"
}